{
  "term_id": "UNKNOWN:0001",
  "gene_name": "Golgin subfamily A member 6-like protein 9",
  "gene": "UniProtKB:A6NEM1",
  "term_label": "Unknown molecular function",
  "gene_symbol": "GOLGA6L9"
}